purine deoxyribonucleoside triphosphate biosynthetic process [GO:0009216] (biological process) Definition: The chemical reactions and pathways resulting in the formation of purine deoxyribonucleoside triphosphate, a compound consisting of a purine base linked to a deoxyribose sugar esterified with triphosphate on the sugar. Sources: GOC:go_curators, ISBN:0198506732 Also known as: purine deoxyribonucleoside triphosphate anabolism, purine deoxyribonucleoside triphosphate biosynthesis, purine deoxyribonucleoside triphosphate formation, purine deoxyribonucleoside triphosphate synthesis Relationships: is a type of purine nucleoside triphosphate biosynthetic process [GO:0009145]; is a type of GO:0009202; is a type of purine deoxyribonucleoside triphosphate metabolic process [GO:0009215] Subtypes: GO:0006175, GO:0046071